{
  "gene_symbol": "CTNNB1",
  "gene": "UniProtKB:P35222",
  "gene_name": "Catenin beta-1",
  "term_label": "cytoplasm",
  "term_id": "GO:0005737"
}